hydrogen sulfide biosynthetic process [GO:0070814] (biological process) Also known as: hydrogen sulfide anabolism, hydrogen sulfide biosynthesis, hydrogen sulfide formation, hydrogen sulfide synthesis, hydrogen sulphide biosynthesis, hydrogen sulphide biosynthetic process Regulation: regulated by GO:1904826; negatively regulated by negative regulation of hydrogen sulfide biosynthetic process [GO:1904827]; positively regulated by GO:1904828 Definition: The chemical reactions and pathways resulting in the formation of hydrogen sulfide, H2S. Relationships: is a type of sulfur compound biosynthetic process [GO:0044272]; is a type of hydrogen sulfide metabolic process [GO:0070813] Sources: GOC:mah